{
  "term_id": "GO:0031267",
  "gene_name": "RILP-like protein 2",
  "gene": "UniProtKB:Q969X0",
  "term_label": "small GTPase binding",
  "gene_symbol": "RILPL2"
}